{
  "term_id": "GO:0006357",
  "gene_symbol": "ZNF286A",
  "gene": "UniProtKB:Q9HBT8",
  "term_label": "regulation of transcription by RNA polymerase II",
  "gene_name": "Zinc finger protein 286A"
}